{
  "term_id": "GO:0006357",
  "term_label": "regulation of transcription by RNA polymerase II",
  "gene": "UniProtKB:P18847",
  "gene_symbol": "ATF3",
  "gene_name": "Cyclic AMP-dependent transcription factor ATF-3"
}